negative regulation of insulin receptor signaling pathway by insulin receptor internalization [GO:0038014] (biological process) Relationships: is a type of GO:0038011; is a type of insulin receptor internalization [GO:0038016]; is_a negative regulation of insulin receptor signaling pathway [GO:0046627] Definition: Any process in which internalization of an insulin receptor stops, prevents, or reduces the frequency, rate or extent of insulin receptor signal transduction. Internalization of insulin in association with its receptor clears insulin from the circulation and is necessary for subsequent insulin dissociation from the receptor and insulin degradation. References: PMID:18492485, PMID:7821727, PMID:7978876, PMID:9609114 Sources: GOC:bf, GOC:signaling Also known as: agonist-stimulated insulin receptor internalization, negative regulation of insulin receptor signalling pathway by insulin receptor internalization